{
  "gene_name": "Synaptotagmin-12",
  "gene_symbol": "SYT12",
  "term_label": "plasma membrane",
  "gene": "UniProtKB:Q8IV01",
  "term_id": "GO:0005886"
}